{
  "term_id": "GO:0060271",
  "gene_name": "Centrosomal protein of 70 kDa",
  "gene_symbol": "CEP70",
  "gene": "UniProtKB:Q8NHQ1",
  "term_label": "cilium assembly"
}